{
  "term_id": "GO:0005886",
  "gene": "UniProtKB:Q6P9F7",
  "gene_symbol": "LRRC8B",
  "term_label": "plasma membrane",
  "gene_name": "Volume-regulated anion channel subunit LRRC8B"
}